{
  "gene": "UniProtKB:P01566",
  "gene_name": "Interferon alpha-10",
  "term_id": "GO:0002250",
  "gene_symbol": "IFNA10",
  "term_label": "adaptive immune response"
}